{
  "gene_symbol": "ZNF630",
  "term_label": "nucleus",
  "term_id": "GO:0005634",
  "gene": "UniProtKB:Q2M218",
  "gene_name": "Zinc finger protein 630"
}